{
  "term_label": "Unknown biological process",
  "gene": "UniProtKB:O14633",
  "gene_name": "Late cornified envelope protein 2B",
  "term_id": "UNKNOWN:0002",
  "gene_symbol": "LCE2B"
}